{
  "gene_symbol": "TDRD15",
  "gene": "UniProtKB:B5MCY1",
  "gene_name": "Tudor domain-containing protein 15",
  "term_label": "Unknown molecular function",
  "term_id": "UNKNOWN:0001"
}